regulation of syncytium formation by plasma membrane fusion [GO:0060142] (biological process) Relationships: is a type of regulation of developmental process [GO:0050793]; is_a GO:0051128; regulates syncytium formation by plasma membrane fusion [GO:0000768] Sources: GOC:dph Subtypes: regulation of macrophage fusion [GO:0034239], GO:0034242, positive regulation of syncytium formation by plasma membrane fusion [GO:0060143], GO:1901739 Definition: Any process that modulates the frequency, rate or extent of the formation of a syncytium, a mass of cytoplasm containing several nuclei enclosed within a single plasma membrane, by the fusion of the plasma membranes of two or more individual cells.